{
  "gene_name": "NKAP-like protein",
  "gene": "UniProtKB:Q5M9Q1",
  "gene_symbol": "NKAPL",
  "term_label": "Unknown molecular function",
  "term_id": "UNKNOWN:0001"
}